{
  "gene_symbol": "OR51A7",
  "gene": "UniProtKB:Q8NH64",
  "term_id": "GO:0005886",
  "term_label": "plasma membrane",
  "gene_name": "Olfactory receptor 51A7"
}